palmitoyltransferase complex [GO:0002178] (cellular component) Subtypes: homodimeric serine palmitoyltransferase complex [GO:0002179], serine palmitoyltransferase complex [GO:0017059], GO:0031211, GO:1905961 Definition: A protein complex with palmitoyltransferase activity. Sources: GOC:hjd Relationships: is a type of GO:1990234